glial cell migration in posterior lateral line nerve [GO:0048930] (biological process) Definition: The movement of a glial cell along the axons in the posterior lateral line nerve. Relationships: is_a lateral line nerve glial cell migration [GO:0048896]; is part of posterior lateral line nerve development [GO:0048918] References: PMID:12062041